{
  "term_label": "ribosomal small subunit assembly",
  "gene_name": "Periodic tryptophan protein 2 homolog",
  "gene_symbol": "PWP2",
  "gene": "UniProtKB:Q15269",
  "term_id": "GO:0000028"
}